{
  "term_label": "early endosome membrane",
  "gene_name": "Sorting nexin-20",
  "gene_symbol": "SNX20",
  "gene": "UniProtKB:Q7Z614",
  "term_id": "GO:0031901"
}